pyridine catabolic process [GO:0046221] (biological process) Relationships: is a type of GO:0072526 Also known as: pyridine breakdown, pyridine catabolism, pyridine degradation Sources: GOC:ai Definition: The chemical reactions and pathways resulting in the breakdown of pyridine, a nitrogenous base (C5H5N) obtained from the distillation of bone oil or coal tar, and by the decomposition of certain alkaloids, as a colorless liquid with a peculiar pungent odor.